{
  "term_id": "UNKNOWN:0001",
  "gene_symbol": "CTTN",
  "gene": "UniProtKB:Q14247",
  "gene_name": "Src substrate cortactin",
  "term_label": "Unknown molecular function"
}